tRNA metabolic process [GO:0006399] (biological process) Sources: ISBN:0198506732 Definition: The chemical reactions and pathways involving tRNA, transfer RNA, a class of relatively small RNA molecules responsible for mediating the insertion of amino acids into the sequence of nascent polypeptide chains during protein synthesis. Transfer RNA is characterized by the presence of many unusual minor bases, the function of which has not been completely established. Regulation: regulated by regulation of tRNA metabolic process [GO:1903326]; negatively regulated by negative regulation of tRNA metabolic process [GO:1903327]; positively regulated by positive regulation of tRNA metabolic process [GO:1903328] Relationships: is a type of RNA metabolic process [GO:0016070] Also known as: tRNA metabolism Subtypes: GO:0008033, tRNA transcription [GO:0009304], tRNA decay [GO:0016078], tRNA end turnover [GO:0042778], tRNA aminoacylation [GO:0043039], tRNA threonylcarbamoyladenosine metabolic process [GO:0070525], GO:0106074